{
  "term_label": "Unknown biological process",
  "gene": "UniProtKB:P49356",
  "gene_symbol": "FNTB",
  "term_id": "UNKNOWN:0002",
  "gene_name": "Protein farnesyltransferase subunit beta"
}